{
  "gene_name": "Protein mono-ADP-ribosyltransferase PARP11",
  "term_id": "GO:0005634",
  "gene_symbol": "PARP11",
  "gene": "UniProtKB:Q9NR21",
  "term_label": "nucleus"
}